{
  "term_id": "UNKNOWN:0002",
  "term_label": "Unknown biological process",
  "gene": "UniProtKB:Q9NRJ4",
  "gene_name": "Tubby-related protein 4",
  "gene_symbol": "TULP4"
}